{
  "term_id": "GO:0051015",
  "gene_name": "Protein Shroom4",
  "gene": "UniProtKB:Q9ULL8",
  "term_label": "actin filament binding",
  "gene_symbol": "SHROOM4"
}